{
  "term_id": "GO:0030166",
  "term_label": "proteoglycan biosynthetic process",
  "gene_name": "Carbohydrate sulfotransferase 11",
  "gene": "UniProtKB:Q9NPF2",
  "gene_symbol": "CHST11"
}